{
  "gene": "UniProtKB:Q12840",
  "term_id": "GO:0048489",
  "term_label": "synaptic vesicle transport",
  "gene_symbol": "KIF5A",
  "gene_name": "Kinesin heavy chain isoform 5A"
}